{
  "gene": "UniProtKB:Q96J02",
  "gene_symbol": "ITCH",
  "term_id": "GO:0061630",
  "gene_name": "E3 ubiquitin-protein ligase Itchy homolog",
  "term_label": "ubiquitin protein ligase activity"
}